{
  "gene_name": "Rab11 family-interacting protein 1",
  "gene_symbol": "RAB11FIP1",
  "term_label": "regulated exocytosis",
  "gene": "UniProtKB:Q6WKZ4",
  "term_id": "GO:0045055"
}